{
  "gene": "UniProtKB:Q8NCC3",
  "gene_symbol": "PLA2G15",
  "gene_name": "Phospholipase A2 group XV",
  "term_label": "phosphatidylcholine metabolic process",
  "term_id": "GO:0046470"
}